anaerobic purine nucleobase catabolic process [GO:0019653] (biological process) Relationships: is a type of fermentation [GO:0006113]; is a type of purine nucleobase catabolic process [GO:0006145] Sources: GOC:mah Also known as: anaerobic purine base catabolic process, anaerobic purine base catabolism, purine base fermentation, anaerobic purine catabolic process, purine fermentation Definition: The anaerobic chemical reactions and pathways resulting in the breakdown of purine nucleobases, yielding energy in the form of ATP.